{
  "gene_name": "Putative zinc finger protein 705B",
  "term_id": "GO:0006357",
  "term_label": "regulation of transcription by RNA polymerase II",
  "gene": "UniProtKB:P0CI00",
  "gene_symbol": "ZNF705B"
}